{
  "term_label": "Unknown molecular function",
  "gene_name": "Tumor necrosis factor alpha-induced protein 8-like protein 1",
  "gene": "UniProtKB:Q8WVP5",
  "gene_symbol": "TNFAIP8L1",
  "term_id": "UNKNOWN:0001"
}